{
  "term_label": "kinase binding",
  "term_id": "GO:0019900",
  "gene": "UniProtKB:Q6AWC2",
  "gene_name": "Protein WWC2",
  "gene_symbol": "WWC2"
}